{
  "gene_name": "Cathepsin B",
  "term_label": "lysosome",
  "gene": "UniProtKB:P07858",
  "gene_symbol": "CTSB",
  "term_id": "GO:0005764"
}